{
  "term_label": "sprouting angiogenesis",
  "term_id": "GO:0002040",
  "gene_symbol": "FLT1",
  "gene_name": "Vascular endothelial growth factor receptor 1",
  "gene": "UniProtKB:P17948"
}